{
  "term_label": "Unknown cellular component",
  "gene": "UniProtKB:O60687",
  "gene_symbol": "SRPX2",
  "gene_name": "Sushi repeat-containing protein SRPX2",
  "term_id": "UNKNOWN:0003"
}